amylin receptor activity [GO:0097643] (molecular function) References: PMID:10871296, PMID:12037140, PMID:18687416 Sources: GOC:bhm Definition: Combining with amylin to initiate a change in cell activity. Relationships: is a type of GO:0097642